positive adaptation of signaling pathway [GO:0023059] (biological process) Definition: The positive regulation of a signal transduction pathway in response to a stimulus upon prolonged exposure to that stimulus. Sources: GOC:mtg_signal Also known as: positive adaptation of signalling pathway Relationships: is a type of positive regulation of signal transduction [GO:0009967]; is a type of adaptation of signaling pathway [GO:0023058]